{
  "gene": "UniProtKB:Q6UX73",
  "gene_name": "UPF0764 protein C16orf89",
  "gene_symbol": "C16orf89",
  "term_label": "cytosol",
  "term_id": "GO:0005829"
}